positive regulation of glomerular mesangial cell proliferation [GO:0072126] (biological process) Relationships: is a type of GO:0072124; is a type of positive regulation of cell proliferation involved in kidney development [GO:1901724]; positively regulates GO:0072110 Definition: Any process that increases the frequency, rate or extent of glomerular mesangial cell proliferation. Subtypes: positive regulation of glomerular metanephric mesangial cell proliferation [GO:0072303], positive regulation of mesonephric glomerular mesangial cell proliferation [GO:2000092] Sources: GOC:mtg_kidney_jan10